{
  "gene_symbol": "MTRFR",
  "term_id": "UNKNOWN:0002",
  "gene_name": "Mitochondrial translation release factor in rescue",
  "gene": "UniProtKB:Q9H3J6",
  "term_label": "Unknown biological process"
}